{
  "gene_name": "AF4_FMR2 family member 3",
  "gene_symbol": "AFF3",
  "term_id": "GO:0006355",
  "term_label": "regulation of DNA-templated transcription",
  "gene": "UniProtKB:P51826"
}